{
  "gene_name": "Leucine-rich repeat serine_threonine-protein kinase 2",
  "term_id": "GO:0005886",
  "term_label": "plasma membrane",
  "gene": "UniProtKB:Q5S007",
  "gene_symbol": "LRRK2"
}